extracellular membraneless organelle [GO:0043264] (cellular component) Sources: GOC:jl Definition: Organized structure of distinctive morphology and function, not bounded by a lipid bilayer membrane and occurring outside the cell. Relationships: is a type of GO:0043228; is a type of extracellular organelle [GO:0043230] Subtypes: cellulosome [GO:0043263], trichocyst [GO:0055039], GO:0085026, neutrophil extracellular trap [GO:0140644] Also known as: extracellular non-membrane-bounded organelle, extracellular non-membrane-enclosed organelle